{
  "gene_name": "C-X-C motif chemokine 11",
  "gene_symbol": "CXCL11",
  "term_id": "UNKNOWN:0003",
  "gene": "UniProtKB:O14625",
  "term_label": "Unknown cellular component"
}